{
  "term_label": "plasma membrane",
  "gene_name": "Transient receptor potential cation channel subfamily V member 4",
  "term_id": "GO:0005886",
  "gene": "UniProtKB:Q9HBA0",
  "gene_symbol": "TRPV4"
}